{
  "term_label": "voltage-gated potassium channel complex",
  "gene_symbol": "KCNA6",
  "term_id": "GO:0008076",
  "gene_name": "Potassium voltage-gated channel subfamily A member 6",
  "gene": "UniProtKB:P17658"
}